{
  "gene_symbol": "CD1B",
  "gene_name": "T-cell surface glycoprotein CD1b",
  "term_label": "antigen processing and presentation, endogenous lipid antigen via MHC class Ib",
  "term_id": "GO:0048006",
  "gene": "UniProtKB:P29016"
}